{
  "gene": "UniProtKB:A2RUT3",
  "term_id": "UNKNOWN:0002",
  "gene_name": "Transmembrane protein 89",
  "term_label": "Unknown biological process",
  "gene_symbol": "TMEM89"
}